plant-type ovary development [GO:0035670] (biological process) Definition: The process whose specific outcome is the progression of an ovary that produces an ovule over time, from its formation to the mature structure. The ovary is the enlarged basal portion of a carpel and matures into a fruit. An ovule is the multicellular structure that gives rise to and contains the female reproductive cells, and develops into a seed. Relationships: is a type of reproductive structure development [GO:0048608]; is part of carpel development [GO:0048440] Sources: GOC:bf, GOC:tb, ISBN:0879015322